{
  "term_id": "GO:0003735",
  "gene_name": "Large ribosomal subunit protein uL23",
  "gene": "UniProtKB:P62750",
  "term_label": "structural constituent of ribosome",
  "gene_symbol": "RPL23A"
}